quinine 3-monooxygenase activity [GO:0050591] (molecular function) Sources: EC:1.14.14.55, RHEA:20149 Definition: Catalysis of the reaction: H+ + NADPH + O2 + quinine = 3-hydroxyquinine + H2O + NADP+. Also known as: quinine 3-hydroxylase activity, nifedipine oxidase activity, quinine,NADPH:oxygen oxidoreductase activity Relationships: is a type of oxidoreductase activity, acting on paired donors, with incorporation or reduction of molecular oxygen, NAD(P)H as one donor, and incorporation of one atom of oxygen [GO:0016709]